{
  "term_label": "Unknown cellular component",
  "gene": "UniProtKB:Q8TD35",
  "term_id": "UNKNOWN:0003",
  "gene_name": "Protein LKAAEAR1",
  "gene_symbol": "LKAAEAR1"
}